{
  "gene_name": "Zinc finger protein 42 homolog",
  "term_id": "GO:0000978",
  "term_label": "RNA polymerase II cis-regulatory region sequence-specific DNA binding",
  "gene_symbol": "ZFP42",
  "gene": "UniProtKB:Q96MM3"
}